{
  "gene": "UniProtKB:A0A075B759",
  "gene_symbol": "PPIAL4E",
  "term_label": "peptidyl-prolyl cis-trans isomerase activity",
  "gene_name": "Peptidyl-prolyl cis-trans isomerase A-like 4E",
  "term_id": "GO:0003755"
}